{
  "term_label": "cytoplasm",
  "term_id": "GO:0005737",
  "gene_symbol": "LHPP",
  "gene": "UniProtKB:Q9H008",
  "gene_name": "Phospholysine phosphohistidine inorganic pyrophosphate phosphatase"
}